{
  "term_id": "UNKNOWN:0003",
  "gene_name": "Dehydrogenase_reductase SDR family member 1",
  "term_label": "Unknown cellular component",
  "gene": "UniProtKB:Q96LJ7",
  "gene_symbol": "DHRS1"
}